threonine-tRNA ligase activity [GO:0004829] (molecular function) Definition: Catalysis of the reaction: ATP + L-threonine + tRNA(Thr) = AMP + diphosphate + L-threonyl-tRNA(Thr). Also known as: threonyl-tRNA synthetase activity, L-threonine:tRNAThr ligase (AMP-forming), TRS, threonine translase activity, threonine-transfer ribonucleate synthetase activity, threonyl ribonucleic synthetase activity, threonyl-transfer RNA synthetase activity, threonyl-transfer ribonucleate synthetase activity, threonyl-transfer ribonucleic acid synthetase activity Sources: EC:6.1.1.3 Relationships: is a type of GO:0004812